{
  "gene": "UniProtKB:Q8WXR4",
  "term_id": "GO:0051491",
  "gene_name": "Myosin-IIIb",
  "gene_symbol": "MYO3B",
  "term_label": "positive regulation of filopodium assembly"
}